{
  "gene": "UniProtKB:Q15696",
  "gene_name": "U2 small nuclear ribonucleoprotein auxiliary factor 35 kDa subunit-related protein 2",
  "term_id": "GO:0030628",
  "gene_symbol": "ZRSR2",
  "term_label": "pre-mRNA 3'-splice site binding"
}